{
  "gene": "UniProtKB:Q6NWY9",
  "term_id": "GO:0000398",
  "term_label": "mRNA splicing, via spliceosome",
  "gene_name": "Pre-mRNA-processing factor 40 homolog B",
  "gene_symbol": "PRPF40B"
}